regulation of Hulle cell development [GO:0070808] (biological process) Subtypes: negative regulation of Hulle cell development [GO:0070809], GO:0070810 Definition: Any process that modulates the frequency, rate or extent of Hulle cell development, a process that leads to the formation of Hulle cells. Hulle cells are specialized multinucleate cells that originate from a nest-like aggregation of hyphae during sexual development and serve as nurse cells to the developing cleistothecium, or fruiting body. Relationships: is_a regulation of cell development [GO:0060284]; is a type of GO:2000241; regulates Hulle cell development [GO:0070792] Sources: GOC:mah